{
  "term_id": "UNKNOWN:0001",
  "gene": "UniProtKB:Q6ZVN7",
  "gene_name": "Putative protein SEM1, isoform 2",
  "term_label": "Unknown molecular function",
  "gene_symbol": "SEM1"
}